{
  "gene": "UniProtKB:Q60I27",
  "gene_symbol": "ALS2CL",
  "term_label": "guanyl-nucleotide exchange factor activity",
  "term_id": "GO:0005085",
  "gene_name": "ALS2 C-terminal-like protein"
}